{
  "gene_name": "Signal recognition particle subunit SRP68",
  "term_label": "signal recognition particle, endoplasmic reticulum targeting",
  "gene": "UniProtKB:Q9UHB9",
  "term_id": "GO:0005786",
  "gene_symbol": "SRP68"
}